ADP-ribosylserine hydrolase activity [GO:0140292] (molecular function) Definition: Catalysis of the reaction: (ADP-D-ribosyl)-L-seryl-[protein] + H2O = L-seryl-[protein] + ADP-ribose. References: PMID:28650317, PMID:29234005 Sources: RHEA:58256 Relationships: is a type of hydrolase activity, hydrolyzing N-glycosyl compounds [GO:0016799]; is a type of GO:0140096